{
  "gene": "UniProtKB:O95486",
  "gene_symbol": "SEC24A",
  "gene_name": "Protein transport protein Sec24A",
  "term_label": "COPII vesicle coat",
  "term_id": "GO:0030127"
}